{
  "term_label": "Unknown cellular component",
  "term_id": "UNKNOWN:0003",
  "gene_symbol": "IL15RA",
  "gene_name": "Interleukin-15 receptor subunit alpha",
  "gene": "UniProtKB:Q13261"
}